ADP-ribosylglutamate hydrolase activity [GO:0140293] (molecular function) Definition: Catalysis of the reaction: (ADP-D-ribosyl)-L-glutamyl-[protein] + H2O = L-glutamyl-[protein] + ADP-ribose. Relationships: is a type of hydrolase activity, hydrolyzing N-glycosyl compounds [GO:0016799]; is_a GO:0140096 References: PMID:23481255